octopamine or tyramine signaling pathway [GO:0007211] (biological process) Regulation: regulated by regulation of octopamine or tyramine signaling pathway [GO:2000125]; negatively regulated by negative regulation of octopamine or tyramine signaling pathway [GO:2000126]; positively regulated by positive regulation of octopamine or tyramine signaling pathway [GO:2000127] Also known as: octopamine or tyramine signalling pathway, octopamine/tyramine signaling pathway Definition: A G protein-coupled receptor signaling pathway initiated by octopamine or tyramine binding to their receptor on the surface of a target cell, and ending with the regulation of a downstream cellular process, e.g. transcription, and ending with the regulation of a downstream cellular process. Octopamine and tyramine are decarboxylation products of tyrosine, and are the invertebrate counterparts of the vertebrate adrenergic transmitters. References: PMID:15355245 Sources: GOC:mah Subtypes: GO:0071927, GO:0071928 Relationships: is a type of GO:0007186